{
  "term_label": "nucleus",
  "term_id": "GO:0005634",
  "gene": "UniProtKB:Q09019",
  "gene_name": "Dystrophia myotonica WD repeat-containing protein",
  "gene_symbol": "DMWD"
}